{
  "gene_symbol": "RMDN2",
  "gene": "UniProtKB:Q96LZ7",
  "term_label": "cytoplasm",
  "gene_name": "Regulator of microtubule dynamics protein 2",
  "term_id": "GO:0005737"
}